myelin sheath abaxonal region [GO:0035748] (cellular component) Relationships: is a type of GO:0110165; is part of myelin sheath [GO:0043209] References: PMID:20237282 Sources: GOC:BHF Definition: The region of the myelin sheath furthest from the axon.